{
  "gene": "UniProtKB:P78334",
  "term_label": "synaptic transmission, GABAergic",
  "term_id": "GO:0051932",
  "gene_name": "Gamma-aminobutyric acid receptor subunit epsilon",
  "gene_symbol": "GABRE"
}